{
  "term_id": "GO:1990221",
  "gene_symbol": "LYRM4",
  "term_label": "L-cysteine desulfurase complex",
  "gene": "UniProtKB:Q9HD34",
  "gene_name": "LYR motif-containing protein 4"
}